monocyte homeostasis [GO:0035702] (biological process) References: PMID:18832716 Sources: CL:0000576, GOC:BHF Definition: The process of regulating the proliferation and elimination of monocytes such that the total number of monocytes within a whole or part of an organism is stable over time in the absence of an outside stimulus. Relationships: is a type of leukocyte homeostasis [GO:0001776]; is a type of myeloid cell homeostasis [GO:0002262]